{
  "gene_symbol": "GLIS2",
  "gene": "UniProtKB:Q9BZE0",
  "gene_name": "Zinc finger protein GLIS2",
  "term_label": "nucleus",
  "term_id": "GO:0005634"
}